regulation of cardiac muscle tissue growth [GO:0055021] (biological process) Definition: Any process that modulates the frequency, rate or extent of cardiac muscle growth. Subtypes: GO:0055022, positive regulation of cardiac muscle tissue growth [GO:0055023], regulation of cardiac muscle cell proliferation [GO:0060043], regulation of cell growth involved in cardiac muscle cell development [GO:0061050] Relationships: is_a regulation of heart growth [GO:0060420]; regulates cardiac muscle tissue growth [GO:0055017] Sources: GOC:vk